negative regulation of pyrimidine nucleotide biosynthetic process [GO:1900398] (biological process) Sources: GOC:TermGenie Relationships: is a type of negative regulation of nucleotide biosynthetic process [GO:0030809]; is a type of regulation of pyrimidine nucleotide biosynthetic process [GO:1900397]; negatively regulates pyrimidine nucleotide biosynthetic process [GO:0006221] Definition: Any process that stops, prevents or reduces the frequency, rate or extent of pyrimidine nucleotide biosynthetic process. Also known as: down regulation of pyrimidine nucleotide anabolism, down regulation of pyrimidine nucleotide biosynthesis, down regulation of pyrimidine nucleotide biosynthetic process, down regulation of pyrimidine nucleotide formation, down regulation of pyrimidine nucleotide synthesis, down-regulation of pyrimidine nucleotide anabolism, down-regulation of pyrimidine nucleotide biosynthesis, down-regulation of pyrimidine nucleotide biosynthetic process, down-regulation of pyrimidine nucleotide formation, down-regulation of pyrimidine nucleotide synthesis, downregulation of pyrimidine nucleotide anabolism, downregulation of pyrimidine nucleotide biosynthesis, downregulation of pyrimidine nucleotide biosynthetic process, downregulation of pyrimidine nucleotide formation, downregulation of pyrimidine nucleotide synthesis, inhibition of pyrimidine nucleotide anabolism, inhibition of pyrimidine nucleotide biosynthesis, inhibition of pyrimidine nucleotide formation, inhibition of pyrimidine nucleotide synthesis, negative regulation of pyrimidine nucleotide anabolism, negative regulation of pyrimidine nucleotide biosynthesis, negative regulation of pyrimidine nucleotide formation, negative regulation of pyrimidine nucleotide synthesis, inhibition of pyrimidine nucleotide biosynthetic process Subtypes: negative regulation of dCDP biosynthetic process [GO:1903529]